{
  "gene_name": "Casein kinase I isoform alpha-like",
  "gene": "UniProtKB:Q8N752",
  "term_id": "GO:0090090",
  "gene_symbol": "CSNK1A1L",
  "term_label": "negative regulation of canonical Wnt signaling pathway"
}